{
  "gene": "UniProtKB:O95561",
  "term_id": "UNKNOWN:0002",
  "gene_name": "Uncharacterized protein C1orf105",
  "gene_symbol": "C1orf105",
  "term_label": "Unknown biological process"
}